{
  "gene_symbol": "IL36B",
  "gene": "UniProtKB:Q9NZH7",
  "gene_name": "Interleukin-36 beta",
  "term_id": "GO:0005615",
  "term_label": "extracellular space"
}